{
  "gene_symbol": "MFSD6L",
  "term_label": "Unknown biological process",
  "term_id": "UNKNOWN:0002",
  "gene": "UniProtKB:Q8IWD5",
  "gene_name": "Major facilitator superfamily domain-containing protein 6-like"
}